voltage-gated potassium channel activity involved in ventricular cardiac muscle cell action potential repolarization [GO:1902282] (molecular function) Definition: Enables the transmembrane transfer of a potassium ion by a voltage-gated channel through the plasma membrane of a ventricular cardiomyocyte contributing to the repolarization phase of an action potential. A voltage-gated channel is a channel whose open state is dependent on the voltage across the membrane in which it is embedded. Relationships: is a type of voltage-gated potassium channel activity involved in cardiac muscle cell action potential repolarization [GO:0086008]; BFO_0000050 membrane repolarization during ventricular cardiac muscle cell action potential [GO:0098915] Also known as: voltage-dependent potassium channel activity involved in ventricular cardiac muscle cell action potential, voltage-gated potassium ion channel activity involved in ventricular cardiac muscle cell action potential, voltage-sensitive potassium channel involved in ventricular cardiac muscle cell action potential, voltage gated potassium channel activity involved in ventricular cardiac muscle cell action potential References: PMID:8528244 Sources: GOC:BHF, GOC:TermGenie, GOC:mtg_cardiac_conduct_nov11, GOC:rl